{
  "term_label": "meiotic chromosome condensation",
  "gene_name": "Condensin complex subunit 1",
  "gene_symbol": "NCAPD2",
  "term_id": "GO:0010032",
  "gene": "UniProtKB:Q15021"
}